{
  "gene_symbol": "PDE1C",
  "term_id": "GO:0004117",
  "term_label": "calmodulin-activated dual specificity 3',5'-cyclic-GMP, 3',5'-cyclic-AMP phosphodiesterase activity",
  "gene": "UniProtKB:Q14123",
  "gene_name": "Dual specificity calcium_calmodulin-dependent 3',5'-cyclic nucleotide phosphodiesterase 1C"
}